{
  "term_id": "UNKNOWN:0002",
  "gene_name": "Proline-rich transmembrane protein 3",
  "gene_symbol": "PRRT3",
  "gene": "UniProtKB:Q5FWE3",
  "term_label": "Unknown biological process"
}